{
  "gene_symbol": "MAST2",
  "gene": "UniProtKB:Q6P0Q8",
  "gene_name": "Microtubule-associated serine_threonine-protein kinase 2",
  "term_label": "cytoskeleton organization",
  "term_id": "GO:0007010"
}